rhombomere 3 formation [GO:0021660] (BP) Definition: The process that gives rise to rhombomere 3. This process pertains to the initial formation of a structure from unspecified parts. Rhombomeres are transverse segments of the developing rhombencephalon. Rhombomeres are lineage restricted, express different genes from one another, and adopt different developmental fates. Rhombomeres are numbered in anterior to posterior order. Sources: GOC:cls, GOC:curators, GOC:dgh, GOC:dph, GOC:jid Relationships: is a type of GO:0021594; is part of rhombomere 3 morphogenesis [GO:0021658]